{
  "gene_symbol": "SERPINA3",
  "term_label": "response to cytokine",
  "gene_name": "Alpha-1-antichymotrypsin",
  "gene": "UniProtKB:P01011",
  "term_id": "GO:0034097"
}